negative regulation of hormone metabolic process [GO:0032351] (biological process) Also known as: down regulation of hormone metabolic process, down-regulation of hormone metabolic process, downregulation of hormone metabolic process, negative regulation of hormone metabolism, inhibition of hormone metabolic process Subtypes: negative regulation of hormone biosynthetic process [GO:0032353], negative regulation of juvenile hormone metabolic process [GO:0045928], negative regulation of peptide hormone processing [GO:0060570], GO:0090356, negative regulation of retinoic acid biosynthetic process [GO:1900053], negative regulation of thyroid hormone generation [GO:2000610] Relationships: is a type of negative regulation of metabolic process [GO:0009892]; is a type of regulation of hormone metabolic process [GO:0032350]; negatively regulates hormone metabolic process [GO:0042445] Sources: GOC:mah Definition: Any process that stops, prevents, or reduces the frequency, rate or extent of the chemical reactions and pathways involving any hormone.